regulation of vascular associated smooth muscle cell differentiation involved in phenotypic switching [GO:1905930] (biological process) Subtypes: negative regulation of vascular associated smooth muscle cell differentiation involved in phenotypic switching [GO:1905931], positive regulation of vascular associated smooth muscle cell differentiation involved in phenotypic switching [GO:1905932] Also known as: regulation of VSMC differentiation involved in phenotypic switching, regulation of vascular smooth muscle cell differentiation involved in phenotypic switching, regulation of VSMC differentiation involved in phenotypic dimorphism, regulation of vascular associated smooth muscle cell differentiation involved in phenotypic dimorphism, regulation of vascular smooth muscle cell differentiation involved in phenotypic dimorphism References: PMID:25089138 Sources: GOC:BHF, GOC:BHF_miRNA, GOC:TermGenie, GOC:rph, GO_REF:0000058 Definition: Any process that modulates the frequency, rate or extent of vascular smooth muscle cell differentiation involved in phenotypic switching. Relationships: is a type of regulation of vascular associated smooth muscle cell differentiation [GO:1905063]; is a type of GO:1905915; regulates vascular associated smooth muscle cell differentiation involved in phenotypic switching [GO:1905420]